{
  "gene": "UniProtKB:Q14690",
  "term_label": "Unknown biological process",
  "gene_name": "Protein RRP5 homolog",
  "gene_symbol": "PDCD11",
  "term_id": "UNKNOWN:0002"
}